{
  "term_label": "antigen processing and presentation of endogenous peptide antigen via MHC class Ib",
  "gene": "UniProtKB:P10321",
  "gene_symbol": "HLA-C",
  "term_id": "GO:0002476",
  "gene_name": "HLA class I histocompatibility antigen, C alpha chain"
}